type III hypersensitivity [GO:0001802] (biological process) Sources: GOC:add, ISBN:0781735149 Definition: An inflammatory response resulting from recognition of immune complexes via complement or Fc receptors on effector cells leading to activation of neutrophils and other leukocytes and damage to bystander tissue. Note: Note that the Arthus reaction is an example of type III hypersensitivity. Regulation: regulated by regulation of type III hypersensitivity [GO:0001803]; negatively regulated by GO:0001804; positively regulated by GO:0001805 Relationships: is a type of myeloid leukocyte mediated immunity [GO:0002444]; is a type of GO:0002524; is a type of immunoglobulin mediated immune response [GO:0016064]